{
  "term_label": "developmental process",
  "gene_symbol": "TCF23",
  "gene": "UniProtKB:Q7RTU1",
  "term_id": "GO:0032502",
  "gene_name": "Transcription factor 23"
}